metanephric descending thin limb development [GO:0072220] (biological process) Sources: GOC:mtg_kidney_jan10 Definition: The process whose specific outcome is the progression of the metanephric descending thin limb over time, from its formation to the mature structure. The metanephric descending thin limb is a part of the metanephric loop of Henle situated just after the proximal straight tubule (S3). It extends to the tip of the metanephric loop of Henle. Relationships: is a type of descending thin limb development [GO:0072022]; is part of GO:0072236